{
  "term_id": "GO:0000226",
  "gene": "UniProtKB:A6NHL2",
  "term_label": "microtubule cytoskeleton organization",
  "gene_symbol": "TUBAL3",
  "gene_name": "Tubulin alpha chain-like 3"
}